{
  "term_label": "regulation of transcription by RNA polymerase II",
  "gene": "UniProtKB:Q8N8J6",
  "gene_symbol": "ZNF615",
  "term_id": "GO:0006357",
  "gene_name": "Zinc finger protein 615"
}